{
  "term_id": "GO:0015020",
  "gene_name": "Exostosin-like 1",
  "gene_symbol": "EXTL1",
  "gene": "UniProtKB:Q92935",
  "term_label": "glucuronosyltransferase activity"
}